translocation of molecules into host [GO:0044417] (biological process) Subtypes: translocation of peptides or proteins into host [GO:0042000] Also known as: translocation of molecules into other organism during symbiotic interaction, translocation of molecules into other organism involved in symbiotic interaction, transport of molecules into other organism during symbiotic interaction, transport of molecules into host Relationships: is_a biological process involved in interaction with host [GO:0051701] Definition: The directed movement of a molecule(s) produced by an organism to a location inside its host organism. The host is defined as the larger of the organisms involved in a symbiotic interaction. References: PMID:18406478 Sources: GOC:cc